orthogonal array [GO:1990014] (cellular component) Also known as: orthogonal array of particles, OAP, square array Definition: Square array of closely spaced intramembrane particles, 4-6 nm in size, that form supramolecular aggregates found in the plasma membrane of astrocytes, skeletal muscle and epithelial cells. They have been shown to contain aquaporins (water channels). References: PMID:22718347 Sources: NIF_Subcellular:sao1747012216 Relationships: is a type of GO:0110165; is part of GO:0005886